{
  "gene": "UniProtKB:P02675",
  "gene_symbol": "FGB",
  "gene_name": "Fibrinogen beta chain",
  "term_id": "GO:0031012",
  "term_label": "extracellular matrix"
}